{
  "term_id": "UNKNOWN:0002",
  "gene_name": "Regulator of cell cycle RGCC",
  "term_label": "Unknown biological process",
  "gene": "UniProtKB:Q9H4X1",
  "gene_symbol": "RGCC"
}